{
  "term_label": "inner dynein arm assembly",
  "gene_name": "Dynein axonemal assembly factor 5",
  "gene_symbol": "DNAAF5",
  "term_id": "GO:0036159",
  "gene": "UniProtKB:Q86Y56"
}